{
  "term_id": "GO:0051959",
  "gene": "UniProtKB:Q8NCM8",
  "gene_name": "Cytoplasmic dynein 2 heavy chain 1",
  "gene_symbol": "DYNC2H1",
  "term_label": "dynein light intermediate chain binding"
}